{
  "gene": "UniProtKB:Q9Y4W2",
  "term_id": "GO:0000460",
  "gene_symbol": "LAS1L",
  "gene_name": "Ribosomal biogenesis protein LAS1L",
  "term_label": "maturation of 5.8S rRNA"
}